regulation of ATF6-mediated unfolded protein response [GO:1903891] (biological process) Definition: Any process that modulates the frequency, rate or extent of the ATF6-mediated unfolded protein response. Also known as: regulation of ATF6 signal transduction pathway, regulation of ATF6 branch of UPR, regulation of UPR signaling by ATF6 stress sensor, regulation of activating transcription factor 6 signaling in unfolded protein response, regulation of endoplasmic reticulum unfolded protein response; ATF6 signaling, regulation of ATF6-alpha UPR branch, regulation of ATF6-beta UPR branch, regulation of ATF6 signaling in response to endoplasmic reticulum stress Subtypes: negative regulation of ATF6-mediated unfolded protein response [GO:1903892], GO:1903893 Relationships: is a type of regulation of endoplasmic reticulum unfolded protein response [GO:1900101]; regulates ATF6-mediated unfolded protein response [GO:0036500] References: PMID:22013210 Sources: GOC:PARL, GOC:TermGenie, GOC:bf, GO_REF:0000058